acid-amino acid ligase activity [GO:0016881] (molecular function) Definition: Catalysis of the ligation of an acid to an amino acid via a carbon-nitrogen bond, with the concomitant hydrolysis of the diphosphate bond in ATP or a similar triphosphate. Relationships: is a type of ligase activity, forming carbon-nitrogen bonds [GO:0016879] Subtypes: tetrahydrofolylpolyglutamate synthase activity [GO:0004326], glutamate-cysteine ligase activity [GO:0004357], GO:0004363, pantoate-beta-alanine ligase activity [GO:0004592], phosphopantothenate--cysteine ligase activity [GO:0004632], phosphoribosylaminoimidazolesuccinocarboxamide synthase activity [GO:0004639], tubulin-tyrosine ligase activity [GO:0004835], GO:0008716, UDP-N-acetylmuramate-L-alanine ligase activity [GO:0008763], UDP-N-acetylmuramoylalanine-D-glutamate ligase activity [GO:0008764], UDP-N-acetylmuramoylalanyl-D-glutamate-2,6-diaminopimelate ligase activity [GO:0008765], UDP-N-acetylmuramoylalanyl-D-glutamyl-2,6-diaminopimelate-D-alanyl-D-alanine ligase activity [GO:0008766], dihydrofolate synthase activity [GO:0008841], indole-3-acetic acid amido synthetase activity [GO:0010279], L-amino-acid alpha-ligase activity [GO:0034026], coenzyme F420-0 gamma-glutamyl ligase activity [GO:0043773], coenzyme F420-2 alpha-glutamyl ligase activity [GO:0043774], GO:0043860, GO:0047480, D-alanine-alanyl-poly(glycerolphosphate) ligase activity [GO:0047481], UDP-N-acetylmuramoyl-L-alanyl-D-glutamate-L-lysine ligase activity [GO:0047482], GO:0047527, cyclopeptine synthase activity [GO:0047671], carnosine synthase activity [GO:0047730], gamma-glutamylhistamine synthase activity [GO:0047914], homoglutathione synthase activity [GO:0047983], tyrosine-arginine ligase activity [GO:0050367], GO:0050564, GO:0050565, GO:0051108, N-(4-aminobenzoyl)-L-glutamate synthetase activity [GO:0052625], GO:0052626, N-vanillate-L-glutamate synthetase activity [GO:0052627], N-(4-hydroxybenzoyl)-L-glutamate synthetase activity [GO:0052628], L-propargylglycine--L-glutamate ligase activity [GO:0062145], protein-glycine ligase activity [GO:0070735], protein-glutamic acid ligase activity [GO:0070739], GO:0080123, amino acid ligation activity by nonribosomal peptide synthase [GO:0097429], homocarnosine synthase activity [GO:0102102], UDP-N-acetylmuramoyl-L-alanyl-D-glutamate--D-lysine ligase activity [GO:0102195], UDP-N-acetylmuramate-L-alanyl-gamma-D-glutamyl-meso-2,6-diaminoheptanedioate ligase activity [GO:0106418], GO:0160222 Also known as: peptide synthase activity Sources: GOC:jl, GOC:mah